oscillatory cAMP signaling [GO:0140676] (biological process) References: PMID:18657484 Relationships: is a type of cell-cell signaling [GO:0007267]; has part GO:0004115; has part GO:0140582 Also known as: cAMP relay Definition: Fluctuation in the extracellular cAMP levels due to the alternate activation of adenylate cyclase, which produces cAMP, and phosphodiesterase, which degrades it. Occurs in Dictyostelium during early sorocarp development. Oscillation in signaling result is directional chemotaxis of cells towards the center of the aggregate.